4-hydroxymandelate oxidase activity [GO:0047579] (molecular function) Also known as: (S)-2-hydroxy-2-(4-hydroxyphenyl)acetate:oxygen 1-oxidoreductase activity, L-4-hydroxymandelate oxidase (decarboxylating) Relationships: is a type of oxidoreductase activity, acting on the CH-OH group of donors, oxygen as acceptor [GO:0016899] Sources: EC:1.1.3.19, RHEA:15833 Definition: Catalysis of the reaction: (S)-4-hydroxymandelate + H+ + O2 = 4-hydroxybenzaldehyde + CO2 + H2O2.